auditory receptor cell fate commitment [GO:0009912] (biological process) Sources: GOC:lr Also known as: auditory hair cell fate commitment Definition: The process in which the cellular identity of auditory hair cells is acquired and determined. Relationships: is_a inner ear receptor cell fate commitment [GO:0060120]; is part of inner ear auditory receptor cell differentiation [GO:0042491]